{
  "gene_symbol": "ARL5C",
  "term_id": "GO:0005525",
  "gene": "UniProtKB:A6NH57",
  "term_label": "GTP binding",
  "gene_name": "Putative ADP-ribosylation factor-like protein 5C"
}